regulation of female receptivity, post-mating [GO:0046008] (biological process) Definition: Any process that modulates the receptiveness of a female to male advances subsequent to mating. Sources: GOC:go_curators Relationships: is a type of regulation of female receptivity [GO:0045924] Subtypes: GO:0045434, positive regulation of female receptivity, post-mating [GO:0046009]